dicoumaroyl monocaffeoyl spermidine meta-hydroxylase activity [GO:0072548] (molecular function) Definition: Catalysis of the reaction: dicoumaroyl monocaffeoyl spermidine + NADPH + O2 = monocoumaroyl dicaffeoyl spermidine + NADP+ + H2O. Relationships: is a type of GO:0072533 References: PMID:19779199 Sources: GOC:kad